mesodermal-endodermal cell signaling involved in heart induction [GO:0003132] (biological process) Definition: Any process that mediates the transfer of information from mesodermal cells to endodermal cells that contributes to heart induction. Sources: GOC:mtg_heart Also known as: mesodermal-endodermal cell signalling involved in heart induction Relationships: is a type of mesodermal-endodermal cell signaling [GO:0003131]; is part of GO:0003129